yolk syncytial layer development [GO:0106336] (biological process) References: PMID:29180571 Note: The "yolk syncytial layer" structure can be found in Teleostei, Myxini, Chondrichthyes, Lepisosteiformes and Cephalopoda according. Also known as: YSL development Definition: The progression of the yolk syncytial layer over time, from its initial formation to the mature structure. The yolk syncytial layer is the peripheral layer of the yolk cell including nuclei and non-yolky cytoplasm. Relationships: is_a GO:0048856